branched-chain alpha-ketoacid dehydrogenase complex [GO:0160157] (cellular component) Relationships: is a type of alpha-ketoacid dehydrogenase complex [GO:0045240]; is a type of transferase complex [GO:1990234] Definition: A multi-enzyme complex that catalyzes the oxidative decarboxylation of branched-chain alpha-ketoacids derived from L-leucine, L-isoleucine, and L-valine to branched-chain acyl-CoAs. The complex comprises multiple copies of three enzymes referred to as E1, E2 and E3: branched-chain alpha-ketoacid dehydrogenase (E1, a heterotetramer of two alpha and two beta subunits), dihydrolipoyl transacylase (E2), and dihydrolipoamide dehydrogenase (E3). Additional proteins may also be present. References: PMID:10464218, PMID:10745006, PMID:3593587 Also known as: BCKD complex, BKDH complex Note: The catalytic activities of the individual components of this complex are represented by the molecular function terms '3-methyl-2-oxobutanoate dehydrogenase (2-methylpropanoyl-transferring) activity ; GO:0003863' (E1), 'dihydrolipoyllysine-residue (2-methylpropanoyl)transferase activity ; GO:0043754' (E2), and 'dihydrolipoyl dehydrogenase activity ; GO:0004148' (E3).